protein carboxyl O-methyltransferase activity [GO:0051998] (molecular function) Sources: GOC:ai Definition: Catalysis of the transfer of a methyl group to a carboxyl group on a protein. Subtypes: protein C-terminal carboxyl O-methyltransferase activity [GO:0003880], protein-L-isoaspartate (D-aspartate) O-methyltransferase activity [GO:0004719], GO:0008983 Relationships: is_a GO:0008276; is a type of carboxyl-O-methyltransferase activity [GO:0010340] Also known as: protein carboxyl methyltransferase activity